{
  "gene": "UniProtKB:P03905",
  "gene_symbol": "MT-ND4",
  "gene_name": "NADH-ubiquinone oxidoreductase chain 4",
  "term_id": "GO:0009060",
  "term_label": "aerobic respiration"
}